fructosyltransferase activity [GO:0050738] (molecular function) Subtypes: 6G-fructosyltransferase activity [GO:0033841], 1,2-beta-fructan 1F-fructosyltransferase activity [GO:0047207], aldose beta-D-fructosyltransferase activity [GO:0047642], sucrose 1F-fructosyltransferase activity [GO:0050306] Sources: GOC:ai Definition: Catalysis of the transfer of a fructosyl group to an acceptor molecule, typically another carbohydrate or a lipid. Relationships: is a type of GO:0016758